{
  "gene": "UniProtKB:O75473",
  "gene_name": "Leucine-rich repeat-containing G-protein coupled receptor 5",
  "term_label": "positive regulation of canonical Wnt signaling pathway",
  "term_id": "GO:0090263",
  "gene_symbol": "LGR5"
}